{
  "term_label": "Unknown molecular function",
  "gene": "UniProtKB:Q3SXM5",
  "term_id": "UNKNOWN:0001",
  "gene_name": "Inactive hydroxysteroid dehydrogenase-like protein 1",
  "gene_symbol": "HSDL1"
}